{
  "term_id": "GO:0045087",
  "gene_symbol": "TRIM17",
  "gene_name": "E3 ubiquitin-protein ligase TRIM17",
  "gene": "UniProtKB:Q9Y577",
  "term_label": "innate immune response"
}